{
  "gene_name": "Neuronal PAS domain-containing protein 4",
  "gene": "UniProtKB:Q8IUM7",
  "term_label": "DNA-binding transcription factor activity, RNA polymerase II-specific",
  "term_id": "GO:0000981",
  "gene_symbol": "NPAS4"
}